{
  "gene": "UniProtKB:Q92535",
  "gene_symbol": "PIGC",
  "term_label": "glycosylphosphatidylinositol-N-acetylglucosaminyltransferase (GPI-GnT) complex",
  "gene_name": "Phosphatidylinositol N-acetylglucosaminyltransferase subunit C",
  "term_id": "GO:0000506"
}